{
  "gene_symbol": "ZNF221",
  "gene_name": "Zinc finger protein 221",
  "term_id": "GO:0000981",
  "gene": "UniProtKB:Q9UK13",
  "term_label": "DNA-binding transcription factor activity, RNA polymerase II-specific"
}